{
  "gene_symbol": "PRDX2",
  "gene_name": "Peroxiredoxin-2",
  "term_id": "GO:0045454",
  "term_label": "cell redox homeostasis",
  "gene": "UniProtKB:P32119"
}